{
  "gene_symbol": "IFI44",
  "gene": "UniProtKB:Q8TCB0",
  "gene_name": "Interferon-induced protein 44",
  "term_label": "immune response",
  "term_id": "GO:0006955"
}